{
  "term_label": "plasma membrane",
  "gene_symbol": "SPINT1",
  "gene_name": "Kunitz-type protease inhibitor 1",
  "term_id": "GO:0005886",
  "gene": "UniProtKB:O43278"
}